{
  "gene_symbol": "LINC00304",
  "term_id": "UNKNOWN:0002",
  "term_label": "Unknown biological process",
  "gene_name": "Putative uncharacterized protein encoded by LINC00304",
  "gene": "UniProtKB:Q8N9R0"
}